cellular response to low light intensity stimulus [GO:0071487] (biological process) Definition: Any process that results in a change in state or activity of a cell (in terms of movement, secretion, enzyme production, gene expression, etc.) as a result of a low light intensity stimulus. Low light intensity is defined as a level of electromagnetic radiation at or below 0.1 micromols/m2. Relationships: is a type of response to low light intensity stimulus [GO:0009645]; is a type of cellular response to light intensity [GO:0071484] Sources: GOC:mah